{
  "gene": "UniProtKB:Q6PI97",
  "gene_symbol": "HOATZ",
  "term_label": "Unknown cellular component",
  "gene_name": "Cilia- and flagella-associated protein HOATZ",
  "term_id": "UNKNOWN:0003"
}